{
  "gene_symbol": "RPL5",
  "term_label": "structural constituent of ribosome",
  "gene": "UniProtKB:P46777",
  "term_id": "GO:0003735",
  "gene_name": "Large ribosomal subunit protein uL18"
}